{
  "gene": "UniProtKB:Q8IZM0",
  "term_id": "UNKNOWN:0002",
  "gene_symbol": "Q8IZM0",
  "term_label": "Unknown biological process",
  "gene_name": "Putative CNGA1-overlapping antisense gene protein"
}